{
  "gene_symbol": "PSD3",
  "term_id": "GO:0032587",
  "term_label": "ruffle membrane",
  "gene": "UniProtKB:Q9NYI0",
  "gene_name": "PH and SEC7 domain-containing protein 3"
}